lipoxin biosynthetic process [GO:2001301] (biological process) Sources: GOC:mw Subtypes: GO:2001303, lipoxin B4 biosynthetic process [GO:2001306] Relationships: is a type of fatty acid derivative biosynthetic process [GO:1901570] Also known as: lipoxin anabolism, lipoxin biosynthesis, lipoxin formation, lipoxin synthesis Definition: The chemical reactions and pathways resulting in the formation of a lipoxin. A lipoxin is a non-classic eicosanoid and signaling molecule that has four conjugated double bonds and is derived from arachidonic acid.